central B cell anergy [GO:0002341] (biological process) Regulation: regulated by regulation of central B cell anergy [GO:0002914]; negatively regulated by GO:0002915; positively regulated by GO:0002916 Also known as: central B lymphocyte anergy, central B-cell anergy, central B-lymphocyte anergy Definition: Any process contributing to anergy, a state of functional inactivation that occurs as part of tolerance induction, in B cells in the bone marrow. Sources: GOC:jal Relationships: is a type of B cell anergy [GO:0002515]; is part of GO:0002340; is part of central B cell tolerance induction [GO:0002510]